{
  "term_id": "GO:0050776",
  "gene_name": "Caspase recruitment domain-containing protein 10",
  "term_label": "regulation of immune response",
  "gene": "UniProtKB:Q9BWT7",
  "gene_symbol": "CARD10"
}